{
  "gene_name": "WW domain-containing transcription regulator protein 1",
  "gene": "UniProtKB:Q9GZV5",
  "gene_symbol": "WWTR1",
  "term_label": "positive regulation of transcription by RNA polymerase II",
  "term_id": "GO:0045944"
}